{
  "term_id": "GO:0032924",
  "gene_symbol": "ACVR1B",
  "gene_name": "Activin receptor type-1B",
  "gene": "UniProtKB:P36896",
  "term_label": "activin receptor signaling pathway"
}